{
  "gene_name": "Formin-like protein 2",
  "gene": "UniProtKB:Q96PY5",
  "gene_symbol": "FMNL2",
  "term_id": "GO:0016477",
  "term_label": "cell migration"
}